{
  "gene": "UniProtKB:Q14204",
  "gene_symbol": "DYNC1H1",
  "term_label": "nuclear migration",
  "term_id": "GO:0007097",
  "gene_name": "Cytoplasmic dynein 1 heavy chain 1"
}